{
  "gene_symbol": "TAB3",
  "gene": "UniProtKB:Q8N5C8",
  "term_id": "UNKNOWN:0003",
  "gene_name": "TGF-beta-activated kinase 1 and MAP3K7-binding protein 3",
  "term_label": "Unknown cellular component"
}